{
  "term_id": "GO:0030154",
  "term_label": "cell differentiation",
  "gene": "UniProtKB:P49840",
  "gene_symbol": "GSK3A",
  "gene_name": "Glycogen synthase kinase-3 alpha"
}